{
  "gene": "UniProtKB:Q8TAF3",
  "gene_symbol": "WDR48",
  "term_label": "ubiquitin binding",
  "term_id": "GO:0043130",
  "gene_name": "WD repeat-containing protein 48"
}